{
  "gene": "UniProtKB:Q9BYE4",
  "gene_name": "Small proline-rich protein 2G",
  "term_id": "UNKNOWN:0003",
  "gene_symbol": "SPRR2G",
  "term_label": "Unknown cellular component"
}